{
  "term_label": "Cul2-RING ubiquitin ligase complex",
  "term_id": "GO:0031462",
  "gene_name": "PRAME family member 20",
  "gene": "UniProtKB:Q5VT98",
  "gene_symbol": "PRAMEF20"
}